{
  "gene_name": "Zinc finger protein 462",
  "term_id": "GO:0005634",
  "gene_symbol": "ZNF462",
  "term_label": "nucleus",
  "gene": "UniProtKB:Q96JM2"
}